{
  "gene_name": "Endothelial zinc finger protein induced by tumor necrosis factor alpha",
  "gene": "UniProtKB:Q9NQZ8",
  "gene_symbol": "ZNF71",
  "term_id": "GO:0001228",
  "term_label": "DNA-binding transcription activator activity, RNA polymerase II-specific"
}